asparagine-tRNA ligase activity [GO:0004816] (molecular function) Also known as: asparaginyl-tRNA synthetase activity, L-asparagine:tRNAAsn ligase (AMP-forming), asparagine translase activity, asparaginyl transfer RNA synthetase activity, asparaginyl transfer ribonucleic acid synthetase activity, asparaginyl-transfer ribonucleate synthetase activity, asparagyl-transfer RNA synthetase activity Relationships: is a type of aminoacyl-tRNA ligase activity [GO:0004812] Sources: EC:6.1.1.22, RHEA:11180 Definition: Catalysis of the reaction: L-asparagine + ATP + tRNA(Asn) = AMP + Asn-tRNA(Asn) + diphosphate + 2 H+.